{
  "gene_symbol": "IFNLR1",
  "term_id": "GO:0019221",
  "gene_name": "Interferon lambda receptor 1",
  "gene": "UniProtKB:Q8IU57",
  "term_label": "cytokine-mediated signaling pathway"
}